{
  "gene": "UniProtKB:O95837",
  "gene_name": "Guanine nucleotide-binding protein subunit alpha-14",
  "term_label": "G-protein beta/gamma-subunit complex binding",
  "gene_symbol": "GNA14",
  "term_id": "GO:0031683"
}